RNA 2'-phosphatase activity [GO:0160273] (molecular function) References: PMID:36180430 Definition: Catalysis of the reaction: H2O + a 3'-end 2'-phospho-ribonucleotide-RNA = a 3'-end ribonucleotide-RNA + phosphate. Also known as: RNA 2'-Pase activity, Ribonucleic acid 2'-phosphatase activity Relationships: is a type of phosphatase activity [GO:0016791]; is a type of GO:0140098